{
  "gene_symbol": "PAK3",
  "term_label": "regulation of actin cytoskeleton organization",
  "gene": "UniProtKB:O75914",
  "gene_name": "Serine_threonine-protein kinase PAK 3",
  "term_id": "GO:0032956"
}